{
  "gene": "UniProtKB:P43003",
  "term_label": "D-aspartate import across plasma membrane",
  "gene_symbol": "SLC1A3",
  "gene_name": "Excitatory amino acid transporter 1",
  "term_id": "GO:0070779"
}